atrial cardiac muscle cell development [GO:0055014] (biological process) Definition: The process whose specific outcome is the progression of an atrial cardiac muscle cell over time, from its formation to the mature state. Cardiac muscle cells are striated muscle cells that are responsible for heart contraction. The atrium is the part of the heart that receives blood into the organ. Sources: GOC:devbiol Also known as: atrial cardiomyocyte development, atrial heart muscle development Relationships: is a type of cardiac muscle cell development [GO:0055013]; BFO_0000050 atrial cardiac muscle cell differentiation [GO:0055011]